{
  "gene": "UniProtKB:P0C263",
  "term_id": "GO:0000165",
  "gene_name": "Serine_threonine-protein kinase SBK2",
  "term_label": "MAPK cascade",
  "gene_symbol": "SBK2"
}